{
  "gene_name": "Adenomatous polyposis coli protein",
  "term_id": "GO:0008013",
  "term_label": "beta-catenin binding",
  "gene_symbol": "APC",
  "gene": "UniProtKB:P25054"
}